central nervous system myelination [GO:0022010] (biological process) Sources: GOC:cls, GOC:dgh, GOC:dph, GOC:jid, GO_REF:0000021 Relationships: is a type of axon ensheathment in central nervous system [GO:0032291]; is_a myelination [GO:0042552]; is part of oligodendrocyte development [GO:0014003] Definition: The process in which neuronal axons and dendrites become coated with a segmented lipid-rich sheath (myelin) to enable faster and more energetically efficient conduction of electrical impulses. The sheath is formed by the cell membranes of oligodendrocytes in the central nervous system. Adjacent myelin segments are separated by a non-myelinated stretch of axon called a node of Ranvier. Also known as: myelination in central nervous system